bile acid transmembrane transporter activity [GO:0015125] (molecular function) Definition: Enables the transfer of bile acid from one side of a membrane to the other. Bile acids are any of a group of steroid carboxylic acids occurring in bile, where they are present as the sodium salts of their amides with glycine or taurine. Sources: GOC:ai Relationships: is a type of monocarboxylic acid transmembrane transporter activity [GO:0008028]; is a type of GO:0170055; is part of bile acid and bile salt transport [GO:0015721] Subtypes: bile acid:sodium symporter activity [GO:0008508], canalicular bile acid transmembrane transporter activity [GO:0015126], ABC-type bile acid transporter activity [GO:0015432]